{
  "term_id": "UNKNOWN:0003",
  "gene_symbol": "RAB39A",
  "gene": "UniProtKB:Q14964",
  "gene_name": "Ras-related protein Rab-39A",
  "term_label": "Unknown cellular component"
}